{
  "term_id": "UNKNOWN:0002",
  "gene_symbol": "PMS2P11",
  "term_label": "Unknown biological process",
  "gene_name": "Putative postmeiotic segregation increased 2-like protein 11",
  "gene": "UniProtKB:Q13670"
}